{
  "term_label": "Unknown cellular component",
  "gene": "UniProtKB:A0A0A0MTA3",
  "gene_name": "Immunoglobulin kappa joining 5 (Fragment)",
  "gene_symbol": "IGKJ5",
  "term_id": "UNKNOWN:0003"
}